{
  "gene_symbol": "DNAJB7",
  "gene": "UniProtKB:Q7Z6W7",
  "gene_name": "DnaJ homolog subfamily B member 7",
  "term_label": "protein-folding chaperone binding",
  "term_id": "GO:0051087"
}